{
  "gene_symbol": "MAP3K15",
  "term_label": "p38MAPK cascade",
  "gene_name": "Mitogen-activated protein kinase kinase kinase 15",
  "gene": "UniProtKB:Q6ZN16",
  "term_id": "GO:0038066"
}